{
  "term_label": "Unknown molecular function",
  "gene": "UniProtKB:Q9BWC9",
  "term_id": "UNKNOWN:0001",
  "gene_symbol": "CCDC106",
  "gene_name": "Coiled-coil domain-containing protein 106"
}